bacterial-type flagellum basal body, MS ring [GO:0009431] (cellular component) Relationships: is a type of cellular anatomical structure [GO:0110165]; is part of bacterial-type flagellum basal body [GO:0009425] Also known as: flagellar basal body, mounting plate, flagellar basal body, MS ring, flagellin-based flagellum basal body, MS ring References: PMID:10572114, PMID:12624192 Sources: GOC:cilia, GOC:mtg_sensu Definition: One of the rings of the bacterial-type flagellar basal body; a double-flanged ring that anchors the basal body to the cytoplasmic membrane.